transcription factor TFIIIC complex [GO:0000127] (cellular component) Relationships: is a type of RNA polymerase III transcription regulator complex [GO:0090576] Definition: A heterotrimeric transcription factor complex that is involved in regulating transcription from RNA polymerase III (Pol III) promoters. TFIIIC contains three conserved subunits that associate with the proximal Pol III promoter element, and additional subunits that associate with sequence elements downstream of the promoter and are more diverged among species. It also functions as a boundary element to partition genome content into distinct domains outside Pol III promoter regions. References: PMID:11433012, PMID:16751097 Sources: GOC:mah, GOC:vw